spermine transmembrane transporter activity [GO:0000297] (molecular function) Sources: GOC:ai Relationships: is a type of GO:0015203; is part of spermine transmembrane transport [GO:1903710] Definition: Enables the transfer of spermine from one side of a membrane to the other. Spermine is a polybasic amine found in human sperm, in ribosomes and in some viruses, which is involved in nucleic acid packaging. Synthesis is regulated by ornithine decarboxylase which plays a key role in control of DNA replication.